{
  "term_label": "Unknown biological process",
  "gene_name": "Snurportin-1",
  "gene": "UniProtKB:O95149",
  "gene_symbol": "SNUPN",
  "term_id": "UNKNOWN:0002"
}